guanine import across plasma membrane [GO:0098710] (biological process) Definition: The directed movement of guanine from outside of a cell, across the plasma membrane and into the cytosol. Sources: GOC:dos Also known as: guanine import into cell Relationships: is a type of import across plasma membrane [GO:0098739]; is a type of GO:1903716